host-mediated perturbation of viral RNA genome replication [GO:0044830] (biological process) Sources: GOC:jl Definition: A process in which a host organism alters or subverts viral RNA genome replication. Relationships: is a type of host-mediated perturbation of viral process [GO:0044788]; regulates viral RNA genome replication [GO:0039694] Also known as: modulation by host of viral RNA genome replication, regulation by host of viral RNA genome replication